{
  "gene_name": "Interferon kappa",
  "gene": "UniProtKB:Q9P0W0",
  "term_id": "GO:0060337",
  "gene_symbol": "IFNK",
  "term_label": "type I interferon-mediated signaling pathway"
}